{
  "term_id": "GO:0005765",
  "term_label": "lysosomal membrane",
  "gene": "UniProtKB:P28068",
  "gene_name": "HLA class II histocompatibility antigen, DM beta chain",
  "gene_symbol": "HLA-DMB"
}